positive regulation of G2/MI transition of meiotic cell cycle [GO:0110032] (biological process) References: PMID:25492408 Sources: GOC:vw Relationships: is a type of regulation of G2/MI transition of meiotic cell cycle [GO:0110030]; is a type of positive regulation of meiotic cell cycle phase transition [GO:1901995]; is a type of positive regulation of cell cycle G2/M phase transition [GO:1902751]; positively regulates GO:0008315 Definition: Any signaling pathway that activates or increases the activity of a cell cycle cyclin-dependent protein kinase to modulate the switch from G2 phase to MI phase of the meiotic cell cycle.